{
  "gene_symbol": "CIROP",
  "term_label": "Unknown biological process",
  "gene": "UniProtKB:A0A1B0GTW7",
  "term_id": "UNKNOWN:0002",
  "gene_name": "Ciliated left-right organizer metallopeptidase"
}